inositol-1,4,5-trisphosphate 5-phosphatase activity [GO:0052658] (molecular function) Also known as: InsP(3) 5-phosphatase activity, InsP3 5-phosphatase activity, L-myo-inositol 1,4,5-trisphosphate-monoesterase activity, inositol 1,4,5-trisphosphate phosphatase activity, inositol phosphate 5-phosphomonoesterase activity, inositol polyphosphate-5-phosphatase activity, 1D-myo-inositol-1,4,5-trisphosphate 5-phosphohydrolase activity, 5PTase activity, D-myo-inositol 1,4,5-triphosphate 5-phosphatase activity, D-myo-inositol 1,4,5-trisphosphate 5-phosphatase activity, D-myo-inositol(1,4,5)-trisphosphate 5-phosphatase activity, Ins(1,4,5)P3 5-phosphatase activity, inosine triphosphatase activity, myo-inositol-1,4,5-trisphosphate 5-phosphatase activity, type I inositol-polyphosphate phosphatase activity, type II inositol polyphosphate 5-phosphatase activity Sources: RHEA:19797 Relationships: is a type of inositol-polyphosphate 5-phosphatase activity [GO:0004445] Definition: Catalysis of the reaction: 1D-myo-inositol 1,4,5-trisphosphate + H2O = 1D-myo-inositol 1,4-bisphosphate + phosphate.